{
  "gene": "UniProtKB:Q9BYV8",
  "term_id": "UNKNOWN:0001",
  "gene_name": "Centrosomal protein of 41 kDa",
  "term_label": "Unknown molecular function",
  "gene_symbol": "CEP41"
}